{
  "gene_symbol": "SNX10",
  "gene_name": "Sorting nexin-10",
  "term_label": "cilium assembly",
  "term_id": "GO:0060271",
  "gene": "UniProtKB:Q9Y5X0"
}